{
  "term_id": "GO:0005787",
  "gene": "UniProtKB:P67812",
  "gene_name": "Signal peptidase complex catalytic subunit SEC11A",
  "term_label": "signal peptidase complex",
  "gene_symbol": "SEC11A"
}